{
  "term_label": "plasma membrane",
  "gene_name": "Apelin receptor",
  "gene": "UniProtKB:P35414",
  "term_id": "GO:0005886",
  "gene_symbol": "APLNR"
}